chanoclavine-I aldehyde biosynthetic process [GO:1900569] (biological process) Regulation: regulated by regulation of chanoclavine-I aldehyde biosynthetic process [GO:1900646]; negatively regulated by negative regulation of chanoclavine-I aldehyde biosynthetic process [GO:1900647]; positively regulated by positive regulation of chanoclavine-I aldehyde biosynthetic process [GO:1900648] Also known as: chanoclavine-I aldehyde anabolism, chanoclavine-I aldehyde biosynthesis, chanoclavine-I aldehyde formation, chanoclavine-I aldehyde synthesis Sources: GOC:TermGenie, GOC:di Definition: The chemical reactions and pathways resulting in the formation of chanoclavine-I aldehyde. Chanoclavine-I aldehyde is at a branching point in the biosynthetic pathways of fumigaclavine C and ergotamine. Relationships: is a type of ergot alkaloid biosynthetic process [GO:0035837]; is a type of aldehyde biosynthetic process [GO:0046184]; is a type of olefinic compound biosynthetic process [GO:0120255]